{
  "gene": "UniProtKB:P23975",
  "term_label": "dopamine uptake involved in synaptic transmission",
  "gene_symbol": "SLC6A2",
  "term_id": "GO:0051583",
  "gene_name": "Sodium-dependent noradrenaline transporter"
}